{
  "term_label": "inositol phosphate biosynthetic process",
  "gene_symbol": "PPIP5K2",
  "term_id": "GO:0032958",
  "gene_name": "Inositol hexakisphosphate and diphosphoinositol-pentakisphosphate kinase 2",
  "gene": "UniProtKB:O43314"
}